{
  "gene": "UniProtKB:P0CW01",
  "gene_symbol": "TSPY10",
  "gene_name": "Testis-specific Y-encoded protein 10",
  "term_label": "chromatin",
  "term_id": "GO:0000785"
}